{
  "term_label": "U2 snRNP",
  "gene": "UniProtKB:P62316",
  "gene_symbol": "SNRPD2",
  "term_id": "GO:0005686",
  "gene_name": "Small nuclear ribonucleoprotein Sm D2"
}